regulation of autophagosome maturation [GO:1901096] (BP) References: PMID:10436019, PMID:21383079 Sources: GOC:TermGenie, GOC:autophagy Subtypes: negative regulation of autophagosome maturation [GO:1901097], positive regulation of autophagosome maturation [GO:1901098] Also known as: regulation of autophagic vacuole fusion, regulation of autophagosome fusion, regulation of amphisome-lysosome fusion, regulation of autolysosome formation, regulation of fusion of autophagosome with lysosome Relationships: is a type of regulation of macroautophagy [GO:0016241]; is a type of regulation of organelle organization [GO:0033043]; is a type of regulation of protein-containing complex disassembly [GO:0043244]; regulates autophagosome maturation [GO:0097352] Definition: Any process that modulates the frequency, rate or extent of autophagosome maturation.